cellular response to desiccation [GO:0071465] (biological process) Relationships: is a type of GO:0009269; is a type of cellular response to water deprivation [GO:0042631] Definition: Any process that results in a change in state or activity of a cell (in terms of movement, secretion, enzyme production, gene expression, etc.) as a result of a desiccation stimulus, extreme dryness resulting from the prolonged deprivation of water. Also known as: desiccation tolerance Sources: GOC:mah